{
  "term_label": "Unknown molecular function",
  "term_id": "UNKNOWN:0001",
  "gene": "UniProtKB:O95361",
  "gene_name": "Tripartite motif-containing protein 16",
  "gene_symbol": "TRIM16"
}